cardiac cell fate specification [GO:0060912] (biological process) Subtypes: GO:0042685, GO:0061447 Relationships: is_a cell fate specification [GO:0001708]; BFO_0000050 GO:0060911 Also known as: cardiocyte cell fate specification Definition: The process involved in the specification of cardiac cell identity. Once specification has taken place, a cell will be committed to differentiate down a specific pathway if left in its normal environment. Regulation: regulated by regulation of cardiac cell fate specification [GO:2000043]; RO_0002212 by negative regulation of cardiac cell fate specification [GO:2000044] Sources: GOC:mtg_heart